{
  "gene_name": "Hepatoma-derived growth factor",
  "gene_symbol": "HDGF",
  "term_label": "nucleus",
  "gene": "UniProtKB:P51858",
  "term_id": "GO:0005634"
}